negative regulation of meiotic nuclear division [GO:0045835] (biological process) Definition: Any process that stops, prevents, or reduces the frequency, rate or extent of meiosis. Relationships: is a type of GO:0010948; is a type of regulation of meiotic nuclear division [GO:0040020]; is_a GO:0051447; is a type of negative regulation of nuclear division [GO:0051784]; negatively regulates GO:0140013 Also known as: down regulation of meiosis, down-regulation of meiosis, downregulation of meiosis, negative regulation of meiosis, inhibition of meiosis Subtypes: GO:0045128, GO:0051598, GO:0110029, negative regulation of meiotic spindle elongation [GO:1902120] Sources: GOC:go_curators